{
  "term_id": "UNKNOWN:0001",
  "term_label": "Unknown molecular function",
  "gene": "UniProtKB:Q9NRQ5",
  "gene_name": "Single-pass membrane and coiled-coil domain-containing protein 4",
  "gene_symbol": "SMCO4"
}